regulation of bone trabecula formation [GO:1900154] (biological process) Sources: GOC:BHF, GOC:TermGenie Relationships: is a type of regulation of developmental process [GO:0050793]; regulates bone trabecula formation [GO:0060346] Also known as: regulation of bone trabeculation, regulation of skeletal trabecula formation, regulation of skeletal trabeculation, regulation of bone trabecula biogenesis, regulation of skeletal trabecula biogenesis Definition: Any process that modulates the frequency, rate or extent of bone trabecula formation. Subtypes: negative regulation of bone trabecula formation [GO:1900155], positive regulation of bone trabecula formation [GO:1900156]